adaptive immune effector response [GO:0090718] (biological process) Definition: An adaptive immune response that involves one or more immune effector processes and takes place during the effector phase of the adaptive immune response. Subtypes: GO:0090719 Regulation: regulated by regulation of adaptive immune effector response [GO:1905677]; negatively regulated by negative regulation of adaptive immune effector response [GO:1905678]; positively regulated by positive regulation of adaptive immune effector response [GO:1905679] Relationships: is a type of adaptive immune response [GO:0002250]; BFO_0000051 immune effector process [GO:0002252] Sources: GOC:add, ISBN:1405196831